regulation of follicle cell microvillus length [GO:0032533] (biological process) Definition: A process that modulates the length of a microvillus on a follicle cell. Relationships: is a type of regulation of cell size [GO:0008361]; is a type of GO:0032531; is_a regulation of microvillus length [GO:0032532] References: PMID:16260500 Sources: GOC:sart